{
  "term_label": "Unknown molecular function",
  "term_id": "UNKNOWN:0001",
  "gene_name": "PIH1 domain-containing protein 1",
  "gene_symbol": "PIH1D1",
  "gene": "UniProtKB:Q9NWS0"
}